{
  "gene_name": "Fibrinogen alpha chain",
  "gene": "UniProtKB:P02671",
  "term_label": "positive regulation of heterotypic cell-cell adhesion",
  "gene_symbol": "FGA",
  "term_id": "GO:0034116"
}